histone H4 kinase activity [GO:0140997] (molecular function) References: PMID:25303536 Definition: Catalysis of the transfer of a phosphate group to a histone H4. Subtypes: GO:0044023 Relationships: is a type of histone kinase activity [GO:0035173]